in utero embryonic development [GO:0001701] (biological process) Definition: The process whose specific outcome is the progression of the embryo in the uterus over time, from formation of the zygote in the oviduct, to birth. An example of this process is found in Mus musculus. Relationships: is a type of GO:0043009 Sources: GOC:go_curators, GOC:mtg_sensu